{
  "term_label": "4-galactosyl-N-acetylglucosaminide 3-alpha-L-fucosyltransferase activity",
  "gene_symbol": "FUT3",
  "term_id": "GO:0017083",
  "gene_name": "3-galactosyl-N-acetylglucosaminide 4-alpha-L-fucosyltransferase FUT3",
  "gene": "UniProtKB:P21217"
}